myo-inositol phosphate transport [GO:0033271] (biological process) Definition: The directed movement of any phosphorylated myo-inositol into, out of or within a cell, or between cells, by means of some agent such as a transporter or pore. Relationships: is a type of organophosphate ester transport [GO:0015748]; is a type of organic hydroxy compound transport [GO:0015850] Sources: GOC:mah Subtypes: myo-inositol hexakisphosphate transport [GO:0033272]